{
  "term_label": "muscle contraction",
  "term_id": "GO:0006936",
  "gene": "UniProtKB:P07951",
  "gene_name": "Tropomyosin beta chain",
  "gene_symbol": "TPM2"
}